{
  "gene_name": "Ras-related protein Rab-40C",
  "gene": "UniProtKB:Q96S21",
  "term_id": "GO:0006887",
  "gene_symbol": "RAB40C",
  "term_label": "exocytosis"
}